{
  "gene_name": "Protein KPLCE",
  "term_label": "Unknown molecular function",
  "term_id": "UNKNOWN:0001",
  "gene_symbol": "KPLCE",
  "gene": "UniProtKB:Q5T750"
}